{
  "gene_symbol": "GPR39",
  "term_label": "Unknown biological process",
  "gene_name": "G-protein coupled receptor 39",
  "term_id": "UNKNOWN:0002",
  "gene": "UniProtKB:O43194"
}